microglia development [GO:0014005] (biological process) Definition: The process aimed at the progression of a microglial cell over time, from initial commitment of the cell to a specific fate, to the fully functional differentiated cell. Sources: GOC:dgh, GOC:ef Also known as: microglial cell development Relationships: is a type of GO:0021782; is a type of myeloid cell development [GO:0061515]; is part of GO:0014004